{
  "gene": "UniProtKB:Q8WU79",
  "term_id": "GO:0005096",
  "term_label": "GTPase activator activity",
  "gene_symbol": "SMAP2",
  "gene_name": "Stromal membrane-associated protein 2"
}